{
  "gene_symbol": "RALY",
  "gene": "UniProtKB:Q9UKM9",
  "term_id": "GO:0005634",
  "term_label": "nucleus",
  "gene_name": "RNA-binding protein Raly"
}